{
  "term_id": "UNKNOWN:0002",
  "gene": "UniProtKB:Q9Y2K5",
  "gene_symbol": "R3HDM2",
  "gene_name": "R3H domain-containing protein 2",
  "term_label": "Unknown biological process"
}